cytosine/thymine mispair binding [GO:0035488] (MF) Definition: Binding to a double-stranded DNA region containing a C/T mispair. Also known as: C/T mispair binding, T/C mispair binding, thymine/cytosine mispair binding Relationships: is a type of GO:0030983 Sources: GOC:bf, GOC:jh